{
  "gene": "UniProtKB:O75534",
  "term_label": "CRD-mediated mRNA stability complex",
  "gene_symbol": "CSDE1",
  "term_id": "GO:0070937",
  "gene_name": "Cold shock domain-containing protein E1"
}